{
  "gene": "UniProtKB:Q8WVY7",
  "gene_name": "Ubiquitin-like domain-containing CTD phosphatase 1",
  "term_label": "nucleus",
  "term_id": "GO:0005634",
  "gene_symbol": "UBLCP1"
}